{
  "term_label": "3'-5' RNA helicase activity",
  "term_id": "GO:0034458",
  "gene_symbol": "DHX38",
  "gene_name": "Pre-mRNA-splicing factor ATP-dependent RNA helicase PRP16",
  "gene": "UniProtKB:Q92620"
}